{
  "term_id": "UNKNOWN:0002",
  "gene_symbol": "TMEM160",
  "gene": "UniProtKB:Q9NX00",
  "gene_name": "Transmembrane protein 160",
  "term_label": "Unknown biological process"
}